cap-independent translational initiation of circular RNA [GO:0110018] (biological process) Definition: The process where translation initiation recruits the 40S ribosomal subunits in a cap and 5' end independent fashion before an AUG codon is encountered in an appropriate sequence context to initiate circRNA translation. Also known as: cap-independent translational initiation of circRNA References: PMID:28281539, PMID:28344080, PMID:28344082 Sources: GOC:sp Subtypes: IRES-dependent translational initiation of circular RNA [GO:0110019] Relationships: is a type of cap-independent translational initiation [GO:0002190]